{
  "gene_symbol": "RHBG",
  "gene_name": "Ammonium transporter Rh type B",
  "gene": "UniProtKB:Q9H310",
  "term_label": "ammonium homeostasis",
  "term_id": "GO:0097272"
}